{
  "term_id": "GO:0043161",
  "gene_symbol": "ASB1",
  "gene_name": "Ankyrin repeat and SOCS box protein 1",
  "gene": "UniProtKB:Q9Y576",
  "term_label": "proteasome-mediated ubiquitin-dependent protein catabolic process"
}